{
  "gene": "UniProtKB:Q8WUW1",
  "term_label": "regulation of actin polymerization or depolymerization",
  "term_id": "GO:0008064",
  "gene_symbol": "BRK1",
  "gene_name": "Protein BRICK1"
}